detection of hot stimulus involved in thermoception [GO:0120168] (BP) Relationships: is a type of detection of temperature stimulus involved in thermoception [GO:0050960]; is part of sensory perception of hot stimulus [GO:0062036] Definition: The series of events in which a hot stimulus is received and converted into a molecular signal as part of thermoception. References: PMID:21335241 Also known as: sensory detection of heat stimulus during thermoception, sensory detection of hot stimulus during thermoception, sensory transduction of heat stimulus during thermoception, sensory transduction of hot stimulus during thermoception, thermoception, sensory detection of heat stimulus, thermoception, sensory detection of hot stimulus, thermoception, sensory transduction of heat stimulus, thermoception, sensory transduction of hot stimulus